extracellularly glutamate-gated ion channel activity [GO:0005234] (molecular function) Definition: Enables the transmembrane transfer of an ion by a channel that opens when glutamate is bound by the channel complex or one of its constituent parts on the extracellular side of the plasma membrane. Sources: GOC:mtg_transport, ISBN:0815340729 Also known as: extracellular-glutamate-gated ion channel activity Note: Note that this term represents an activity and not a gene product. Consider also annotating to the molecular function term 'glutamate receptor activity ; GO:0008066'. Relationships: is a type of GO:0005231 Subtypes: extracellularly glutamate-gated chloride channel activity [GO:0008068]